histone H3R2 arginine deiminase activity [GO:0140795] (molecular function) References: PMID:15339660 Note: Comment: Note that the residue position corresponds to the canonical human H3 histone (UniProtKB:P84243); this residue is conserved across all eukaryotes. Residue 1 is the first residue following removal of the initiating Methionine (Met). Note that each histone is encoded by multiple genes, and sequences may vary across different genes within an organism. The substrate for histone deiminase may be methyl-arginine, rather than arginine (see PMID:35197210 and PMID:16567635). Also known as: H3-R2 citrullination, histone H3-R2 arginine deiminase activity, histone-arginine deiminase activity (H3-R2 specific) Relationships: is a type of GO:0141057 Definition: Catalysis of the reaction: H2O + histone H3 L-arginyl (position 2)= histone H3 L-citrullyl (position 2) + NH4+, resulting in histone H3 citrullination at position 2.